{
  "term_id": "GO:0005615",
  "term_label": "extracellular space",
  "gene_name": "Acid sphingomyelinase-like phosphodiesterase 3b",
  "gene": "UniProtKB:Q92485",
  "gene_symbol": "SMPDL3B"
}